2-methylcitrate dehydratase activity [GO:0047547] (molecular function) Also known as: (2S,3S)-2-hydroxybutane-1,2,3-tricarboxylate hydro-lyase [(Z)-but-2-ene-1,2,3-tricarboxylate-forming], 2-hydroxybutane-1,2,3-tricarboxylate hydro-lyase activity, 2-methylcitrate hydro-lyase activity, prpD Definition: Catalysis of the reaction: (2S,3S)-2-methylcitrate = cis-2-methylaconitate + H2O. Sources: EC:4.2.1.79, RHEA:17725 Relationships: is_a hydro-lyase activity [GO:0016836]